slow-twitch skeletal muscle fiber contraction [GO:0031444] (biological process) Relationships: is a type of GO:0014721 Sources: GOC:ef, GOC:mah, GOC:mtg_muscle Regulation: regulated by regulation of slow-twitch skeletal muscle fiber contraction [GO:0031449]; negatively regulated by GO:0031450; positively regulated by positive regulation of slow-twitch skeletal muscle fiber contraction [GO:0031451] Also known as: slow-twitch skeletal muscle fibre contraction Definition: A process in which force is generated within slow-twitch skeletal muscle tissue, resulting in a change in muscle geometry. Force generation involves a chemo-mechanical energy conversion step that is carried out by the actin/myosin complex activity, which generates force through ATP hydrolysis. The slow-twitch skeletal muscle is characterized by slow time parameters, low force development and resistance to fatigue.